{
  "gene_symbol": "MARCHF8",
  "gene": "UniProtKB:Q5T0T0",
  "gene_name": "E3 ubiquitin-protein ligase MARCHF8",
  "term_id": "GO:0042287",
  "term_label": "MHC protein binding"
}